inositol phosphoceramide synthase complex [GO:0070916] (cellular component) References: PMID:19726565 Sources: GOC:mah Relationships: is a type of GO:1990234; is part of Golgi apparatus [GO:0005794] Also known as: IPC synthase complex Definition: A protein complex that possesses inositol phosphoceramide synthase activity and contains a catalytic subunit and a regulatory subunit (Aur1p and Kei1p, respectively, in Saccharomyces).